mannosidase activity [GO:0015923] (molecular function) Relationships: is a type of hydrolase activity, hydrolyzing O-glycosyl compounds [GO:0004553] Sources: GOC:ai Definition: Catalysis of the hydrolysis of mannosyl compounds, substances containing a group derived from a cyclic form of mannose or a mannose derivative. Subtypes: alpha-mannosidase activity [GO:0004559], beta-mannosidase activity [GO:0004567], GDP-mannose mannosyl hydrolase activity [GO:0008727]